{
  "term_label": "calcium activated phosphatidylcholine scrambling",
  "term_id": "GO:0061590",
  "gene": "UniProtKB:Q4KMQ2",
  "gene_symbol": "ANO6",
  "gene_name": "Anoctamin-6"
}